{
  "gene": "UniProtKB:P10242",
  "term_label": "mitotic cell cycle",
  "term_id": "GO:0000278",
  "gene_name": "Transcriptional activator Myb",
  "gene_symbol": "MYB"
}